{
  "term_label": "sperm flagellum",
  "gene_name": "Dynein axonemal heavy chain 1",
  "gene": "UniProtKB:Q9P2D7",
  "term_id": "GO:0036126",
  "gene_symbol": "DNAH1"
}